peptidyl-histidine uridylylation [GO:0051114] (BP) Sources: RESID:AA0372 Definition: The uridylylation of peptidyl-histidine to form peptidyl-1'-(phospho-5'-uridine)-L-histidine (otherwise known as tau-UMP-histidine, tele-UMP-histidine) or peptidyl-3'-(phospho-5'-uridine)-L-histidine (otherwise known as pi-UMP-histidine, pros-UMP-histidine). Relationships: is a type of GO:0018177; is a type of peptidyl-histidine modification [GO:0018202]